{
  "gene_name": "Olfactory receptor 10J3",
  "gene": "UniProtKB:Q5JRS4",
  "gene_symbol": "OR10J3",
  "term_id": "GO:0050911",
  "term_label": "detection of chemical stimulus involved in sensory perception of smell"
}